attachment organelle membrane [GO:0033111] (cellular component) Relationships: is_a bounding membrane of organelle [GO:0098588]; is part of attachment organelle [GO:0033099] Sources: GOC:ecd Definition: The lipid bilayer surrounding an attachment organelle. This is a region of the cell membrane facing the environment - in mycoplasma, part of the mycolate outer membrane.